intraciliary transport particle [GO:0030990] (cellular component) Relationships: is a type of protein-containing complex [GO:0032991] Also known as: intraflagellar transport complex, intraflagellar transport particle, IFT complex Note: Note that we deem cilia and microtubule-based flagella to be equivalent. Definition: A nonmembrane-bound oligomeric protein complex that participates in bidirectional transport of molecules (cargo) along axonemal microtubules. References: PMID:14570576, PMID:22118932, PMID:23945166 Sources: GOC:cilia, GOC:kmv